{
  "gene_name": "Myogenin",
  "term_label": "positive regulation of transcription by RNA polymerase II",
  "gene": "UniProtKB:P15173",
  "gene_symbol": "MYOG",
  "term_id": "GO:0045944"
}